{
  "gene": "UniProtKB:A0A1B0GTR4",
  "gene_name": "Putative small proline-rich protein 5",
  "term_label": "Unknown biological process",
  "gene_symbol": "SPRR5",
  "term_id": "UNKNOWN:0002"
}